extrinsic component of external side of cell outer membrane [GO:0031242] (cellular component) Also known as: extrinsic to external leaflet of cell outer membrane, extrinsic to external side of outer membrane, extrinsic to external side of cell outer membrane Relationships: is a type of extrinsic component of cell outer membrane [GO:0031244]; BFO_0000050 external side of cell outer membrane [GO:0031240] Subtypes: extrinsic component of external side of mycolate outer membrane [GO:0036421] Definition: The component of a cell outer membrane consisting of gene products and protein complexes that are loosely bound to its external surface, but not integrated into the hydrophobic region. Sources: GOC:dos, GOC:mah, GOC:mtg_sensu